{
  "term_label": "regulation of transcription by RNA polymerase II",
  "term_id": "GO:0006357",
  "gene": "UniProtKB:P08151",
  "gene_name": "Zinc finger protein GLI1",
  "gene_symbol": "GLI1"
}